{
  "term_id": "GO:0009617",
  "gene_name": "T cell receptor alpha variable 7",
  "gene": "UniProtKB:A0A075B6U4",
  "term_label": "response to bacterium",
  "gene_symbol": "TRAV7"
}